proton-transporting ATP synthase complex [GO:0045259] (cellular component) Definition: A proton-transporting two-sector ATPase complex that catalyzes the phosphorylation of ADP to ATP during oxidative phosphorylation. The complex comprises a membrane sector (F0) that carries out proton transport and a cytoplasmic compartment sector (F1) that catalyzes ATP synthesis by a rotational mechanism; the extramembrane sector (containing 3 a and 3 b subunits) is connected via the d-subunit to the membrane sector by several smaller subunits. Within this complex, the g and e subunits and the 9-12 c subunits rotate by consecutive 120 degree angles and perform parts of ATP synthesis. This movement is driven by the hydrogen ion electrochemical potential gradient. Relationships: is a type of proton-transporting two-sector ATPase complex [GO:0016469]; is a type of GO:0034703; is a type of respiratory chain complex [GO:0098803]; is_a catalytic complex [GO:1902494] Sources: ISBN:0198547684, ISBN:0716743663 Also known as: F1-F0 complex, hydrogen-translocating F-type ATPase complex, hydrogen-transporting ATP synthase complex, proton-transporting F-type ATPase complex